axo-dendritic transport [GO:0008088] (biological process) Subtypes: axonal transport [GO:0098930], GO:0098935, axo-dendritic protein transport [GO:0099640], slow axonal transport [GO:1990832] Definition: The directed movement of organelles or molecules along microtubules in neuron projections. Sources: ISBN:0815316194 Also known as: axon cargo transport, axonal transport, axoplasmic transport Relationships: is a type of transport along microtubule [GO:0010970]; occurs in neuron projection [GO:0043005]